{
  "term_label": "Unknown molecular function",
  "gene_symbol": "MDM4",
  "gene": "UniProtKB:O15151",
  "term_id": "UNKNOWN:0001",
  "gene_name": "Protein Mdm4"
}